hindgut morphogenesis [GO:0007442] (biological process) Definition: The process in which the anatomical structures of the hindgut are generated and organized. Relationships: is a type of anatomical structure morphogenesis [GO:0009653]; is part of digestive tract morphogenesis [GO:0048546]; is part of GO:0061525 Sources: GOC:jid